{
  "gene": "UniProtKB:P50993",
  "gene_name": "Sodium_potassium-transporting ATPase subunit alpha-2",
  "gene_symbol": "ATP1A2",
  "term_label": "cell projection",
  "term_id": "GO:0042995"
}